{
  "gene_name": "Homeobox protein NANOGP8",
  "term_id": "GO:0019827",
  "gene_symbol": "NANOGP8",
  "gene": "UniProtKB:Q6NSW7",
  "term_label": "stem cell population maintenance"
}